nurse cell apoptotic process [GO:0045476] (BP) Definition: Any apoptotic process in a nurse cell. During late oogenesis, following the transfer of substances from the nurse cells to the oocyte, nurse cell remnants are cleared from the egg chamber by apoptotic process. References: PMID:11973306 Sources: CL:0000026, GOC:mtg_apoptosis Also known as: apoptosis of nurse cells, nurse cell programmed cell death by apoptosis, programmed cell death of nurse cells by apoptosis, invertebrate nurse cell apoptosis, nurse cell apoptosis Relationships: is a type of developmental process involved in reproduction [GO:0003006]; is a type of programmed cell death involved in cell development [GO:0010623]; is a type of GO:1902742; is part of oogenesis [GO:0048477] Regulation: regulated by regulation of nurse cell apoptotic process [GO:0045477]; RO_0002212 by negative regulation of nurse cell apoptotic process [GO:0045849]; positively regulated by positive regulation of nurse cell apoptotic process [GO:0045850]